{
  "term_label": "mitochondrial large ribosomal subunit",
  "gene": "UniProtKB:Q9NX20",
  "gene_symbol": "MRPL16",
  "term_id": "GO:0005762",
  "gene_name": "Large ribosomal subunit protein uL16m"
}